{
  "term_id": "UNKNOWN:0001",
  "gene_symbol": "ODR4",
  "gene_name": "Protein odr-4 homolog",
  "term_label": "Unknown molecular function",
  "gene": "UniProtKB:Q5SWX8"
}